{
  "gene": "UniProtKB:P48443",
  "term_label": "RNA polymerase II transcription regulator complex",
  "term_id": "GO:0090575",
  "gene_name": "Retinoic acid receptor RXR-gamma",
  "gene_symbol": "RXRG"
}